{
  "term_label": "Unknown molecular function",
  "term_id": "UNKNOWN:0001",
  "gene": "UniProtKB:A8MWL6",
  "gene_symbol": "A8MWL6",
  "gene_name": "Putative synaptogyrin-2 like protein"
}